{
  "gene_symbol": "FLACC1",
  "gene_name": "Flagellum-associated coiled-coil domain-containing protein 1",
  "term_id": "GO:0005737",
  "term_label": "cytoplasm",
  "gene": "UniProtKB:Q96Q35"
}